{
  "gene": "UniProtKB:Q9H211",
  "term_label": "regulation of DNA-templated DNA replication initiation",
  "gene_name": "DNA replication factor Cdt1",
  "term_id": "GO:0030174",
  "gene_symbol": "CDT1"
}